{
  "term_label": "Unknown cellular component",
  "term_id": "UNKNOWN:0003",
  "gene_name": "Beta-1,3-N-acetylglucosaminyltransferase radical fringe",
  "gene": "UniProtKB:Q9Y644",
  "gene_symbol": "RFNG"
}